{
  "gene_symbol": "CCDC90B",
  "gene_name": "Coiled-coil domain-containing protein 90B, mitochondrial",
  "gene": "UniProtKB:Q9GZT6",
  "term_label": "Unknown molecular function",
  "term_id": "UNKNOWN:0001"
}